{
  "gene": "UniProtKB:Q14028",
  "gene_name": "Cyclic nucleotide-gated cation channel beta-1",
  "term_label": "intracellularly cGMP-activated cation channel activity",
  "term_id": "GO:0005223",
  "gene_symbol": "CNGB1"
}